submerged biofilm formation [GO:0090605] (biological process) Relationships: is a type of biofilm formation [GO:0042710] Also known as: solid substrate biofilm formation Definition: A process in which planktonically growing microorganisms aggregate and grow on solid substrates under the flow of a liquid and produce extracellular polymers that facilitate attachment and matrix formation, resulting in a change in the organisms' growth rate and gene transcription. Sources: GOC:di, GOC:tb Subtypes: GO:0090609